{
  "term_label": "glutaminyl-peptide cyclotransferase activity",
  "term_id": "GO:0016603",
  "gene_symbol": "QPCT",
  "gene": "UniProtKB:Q16769",
  "gene_name": "Glutaminyl-peptide cyclotransferase"
}